central nervous system formation [GO:0021556] (biological process) Definition: The process that gives rise to the central nervous system. This process pertains to the initial formation of a structure from unspecified parts. The central nervous system is the core nervous system that serves an integrating and coordinating function. In vertebrates it consists of the brain, spinal cord and spinal nerves. In those invertebrates with a central nervous system it typically consists of a brain, cerebral ganglia and a nerve cord. Relationships: is a type of anatomical structure formation involved in morphogenesis [GO:0048646]; is part of central nervous system morphogenesis [GO:0021551] Sources: GOC:cls, GOC:dgh, GOC:dph, GOC:jid, GO_REF:0000021